{
  "gene": "UniProtKB:Q5MJ70",
  "gene_symbol": "SPDYA",
  "term_id": "GO:0019901",
  "gene_name": "Speedy protein A",
  "term_label": "protein kinase binding"
}